{
  "gene_symbol": "TWIST1",
  "gene": "UniProtKB:Q15672",
  "gene_name": "Twist-related protein 1",
  "term_id": "UNKNOWN:0003",
  "term_label": "Unknown cellular component"
}